{
  "gene": "UniProtKB:A0A0A0MS03",
  "gene_symbol": "TRBV5-3",
  "gene_name": "Probable non-functional T cell receptor beta variable 5-3",
  "term_id": "GO:0007166",
  "term_label": "cell surface receptor signaling pathway"
}